{
  "term_label": "ubiquitin protein ligase activity",
  "gene_symbol": "TRIM55",
  "term_id": "GO:0061630",
  "gene_name": "Tripartite motif-containing protein 55",
  "gene": "UniProtKB:Q9BYV6"
}